{
  "term_label": "cell surface",
  "term_id": "GO:0009986",
  "gene_symbol": "SIGIRR",
  "gene_name": "Single Ig IL-1-related receptor",
  "gene": "UniProtKB:Q6IA17"
}